pentanamidase activity [GO:0050168] (molecular function) Relationships: is a type of hydrolase activity, acting on carbon-nitrogen (but not peptide) bonds, in linear amides [GO:0016811] Also known as: pentanamide amidohydrolase activity, valeramidase activity Sources: EC:3.5.1.50, RHEA:10000 Definition: Catalysis of the reaction: H2O + pentanamide = NH4 + valerate.